{
  "gene_name": "HEAT repeat-containing protein 5B",
  "gene": "UniProtKB:Q9P2D3",
  "term_label": "intracellular protein localization",
  "gene_symbol": "HEATR5B",
  "term_id": "GO:0008104"
}